{
  "term_id": "UNKNOWN:0001",
  "term_label": "Unknown molecular function",
  "gene_symbol": "LCE1D",
  "gene": "UniProtKB:Q5T752",
  "gene_name": "Late cornified envelope protein 1D"
}